{
  "term_id": "UNKNOWN:0001",
  "gene_name": "Tumor protein p53-inducible nuclear protein 2",
  "gene_symbol": "TP53INP2",
  "term_label": "Unknown molecular function",
  "gene": "UniProtKB:Q8IXH6"
}